poly(hydroxyalkanoate) metabolic process [GO:1901440] (biological process) Subtypes: poly-hydroxybutyrate metabolic process [GO:0042618], GO:1901441 Relationships: is a type of metabolic process [GO:0008152] Definition: The chemical reactions and pathways involving poly(hydroxyalkanoate). Sources: GOC:TermGenie, GOC:mengo_curators Also known as: poly(hydroxyalkanoate) metabolism